3-hydroxypropionyl-CoA dehydratase activity [GO:0043956] (molecular function) Note: Note that this function is one of the activities of the trifunctional enzyme propionyl-coenzyme A synthase. See PMID:11821399. Relationships: is a type of enoyl-CoA hydratase activity [GO:0004300] References: PMID:11821399 Sources: GOC:jl Definition: Catalysis of the reaction: 3-hydroxypropionyl-CoA = acryloyl-CoA + H2O. Also known as: AMP-dependent synthetase and ligase, AMP-dependent synthetase and ligase:Enoyl-CoA hydratase/isomerase, acetyl-coenzyme A synthetase, acetyl-coenzyme A synthetase/GroES-like domain, enoyl-CoA hydratase/isomerase, 3-hydroxy propionyl-CoA dehydratase activity